{
  "gene": "UniProtKB:P05107",
  "term_id": "GO:0008305",
  "term_label": "integrin complex",
  "gene_name": "Integrin beta-2",
  "gene_symbol": "ITGB2"
}